{
  "term_id": "GO:0010813",
  "term_label": "neuropeptide catabolic process",
  "gene_symbol": "LNPEP",
  "gene": "UniProtKB:Q9UIQ6",
  "gene_name": "Leucyl-cystinyl aminopeptidase"
}